{
  "term_id": "GO:0038202",
  "gene_name": "Ribosomal protein S6 kinase alpha-2",
  "term_label": "TORC1 signaling",
  "gene": "UniProtKB:Q15349",
  "gene_symbol": "RPS6KA2"
}